{
  "gene": "UniProtKB:B1ATL7",
  "term_id": "UNKNOWN:0003",
  "term_label": "Unknown cellular component",
  "gene_name": "Proline-rich protein 32",
  "gene_symbol": "PRR32"
}